{
  "gene_symbol": "LAMA3",
  "gene": "UniProtKB:Q16787",
  "term_label": "nervous system development",
  "term_id": "GO:0007399",
  "gene_name": "Laminin subunit alpha-3"
}